{
  "gene_name": "Integrin alpha-3",
  "term_id": "GO:0050900",
  "term_label": "leukocyte migration",
  "gene_symbol": "ITGA3",
  "gene": "UniProtKB:P26006"
}